2-(S)-hydroxypropyl-CoM dehydrogenase activity [GO:0050575] (molecular function) Also known as: 2-(2-(S)-hydroxypropylthio)ethanesulfonate dehydrogenase activity, 2-[2-(S)-hydroxypropylthio]ethanesulfonate:NAD+ oxidoreductase activity Relationships: is a type of GO:0016616 Sources: EC:1.1.1.269, RHEA:21052 Definition: Catalysis of the reaction: 2-(S)-hydroxypropyl-coenzyme M + NAD+ = 2-oxopropyl-coenzyme M + H+ + NADH.